{
  "gene": "UniProtKB:Q96MU6",
  "term_label": "DNA-binding transcription factor activity, RNA polymerase II-specific",
  "gene_name": "Zinc finger protein 778",
  "term_id": "GO:0000981",
  "gene_symbol": "ZNF778"
}